{
  "term_id": "GO:0045271",
  "gene_name": "NADH dehydrogenase [ubiquinone] iron-sulfur protein 7, mitochondrial",
  "gene_symbol": "NDUFS7",
  "term_label": "respiratory chain complex I",
  "gene": "UniProtKB:O75251"
}